2-propylphenol monooxygenase activity [GO:0102322] (molecular function) Relationships: is a type of oxidoreductase activity, acting on paired donors, with incorporation or reduction of molecular oxygen, NAD(P)H as one donor, and incorporation of one atom of oxygen [GO:0016709] Definition: Catalysis of the reaction: 2-propylphenol + O2 + NADH + H+ = 3-propylcatechol + H2O + NAD. Sources: GOC:pz